{
  "gene_name": "Putative protein RFPL3S",
  "gene": "UniProtKB:P0C7P2",
  "gene_symbol": "RFPL3S",
  "term_id": "UNKNOWN:0003",
  "term_label": "Unknown cellular component"
}